{
  "gene_symbol": "DMRT1",
  "term_label": "DNA-binding transcription factor activity, RNA polymerase II-specific",
  "gene": "UniProtKB:Q9Y5R6",
  "term_id": "GO:0000981",
  "gene_name": "Doublesex- and mab-3-related transcription factor 1"
}